{
  "term_label": "Unknown biological process",
  "gene_symbol": "MIX23",
  "gene": "UniProtKB:Q4VC31",
  "gene_name": "Protein MIX23",
  "term_id": "UNKNOWN:0002"
}